{
  "term_label": "cysteine-type deubiquitinase activity",
  "gene_name": "Inactive ubiquitin carboxyl-terminal hydrolase 17-like protein 8",
  "term_id": "GO:0004843",
  "gene_symbol": "USP17L8",
  "gene": "UniProtKB:P0C7I0"
}